{
  "gene_symbol": "STXBP1",
  "gene_name": "Syntaxin-binding protein 1",
  "term_id": "GO:0017075",
  "gene": "UniProtKB:P61764",
  "term_label": "syntaxin-1 binding"
}